membrane protein complex [GO:0098796] (cellular component) Subtypes: mannan polymerase complex [GO:0000136], glycosylphosphatidylinositol-N-acetylglucosaminyltransferase (GPI-GnT) complex [GO:0000506], GO:0000813, ESCRT II complex [GO:0000814], ESCRT III complex [GO:0000815], ER ubiquitin ligase complex [GO:0000835], 5-lipoxygenase complex [GO:0002180], signal recognition particle receptor complex [GO:0005785], GO:0005787, GO:0005942, oligosaccharyltransferase complex [GO:0008250], photosystem [GO:0009521], GO:0009538, GO:0009539, photosystem II oxygen evolving complex [GO:0009654], photosystem I antenna complex [GO:0009782], photosystem II antenna complex [GO:0009783], fatty acid elongase complex [GO:0009923], Toc complex [GO:0010006], chloroplast outer membrane translocon [GO:0010278], proton-transporting two-sector ATPase complex [GO:0016469], sodium ion-transporting two-sector ATPase complex [GO:0016472], meprin A complex [GO:0017090], phycobilisome [GO:0030089], membrane coat [GO:0030117], AP-type membrane coat adaptor complex [GO:0030119], HOPS complex [GO:0030897], retromer complex [GO:0030904], GO:0030905, retromer, cargo-selective complex [GO:0030906], GO:0030964, GO:0031201, endoplasmic reticulum Sec complex [GO:0031205], Sec62/Sec63 complex [GO:0031207], GO:0031502, Tic complex [GO:0031897], SREBP-SCAP complex [GO:0032936], SREBP-SCAP-Insig complex [GO:0032937], endosomal scaffold complex [GO:0032969], GO:0033177, GO:0033178, GO:0033254, protein C inhibitor-acrosin complex [GO:0033282], VCP-NPL4-UFD1 AAA ATPase complex [GO:0034098], Vps55/Vps68 complex [GO:0034424], pre-B cell receptor complex [GO:0035369], Derlin-1-VIMP complex [GO:0036502], Derlin-1 retrotranslocation complex [GO:0036513], GPI-anchor transamidase complex [GO:0042765], MHC class I peptide loading complex [GO:0042824], TAP complex [GO:0042825], UDP-N-acetylglucosamine transferase complex [GO:0043541], starch utilization system complex [GO:0044570], Dsc E3 ubiquitin ligase complex [GO:0044695], respiratory chain complex II (succinate dehydrogenase) [GO:0045273], fumarate reductase complex [GO:0045283], lipopolysaccharide receptor complex [GO:0046696], pore complex [GO:0046930], chaperone-mediated autophagy translocation complex [GO:0061742], GO:0061779, ATG2-ATG18 complex [GO:0062079], GO:0062137, PAS complex [GO:0070772], translocon complex [GO:0071256], clathrin complex [GO:0071439], Nem1-Spo7 phosphatase complex [GO:0071595], Ragulator complex [GO:0071986], EMC complex [GO:0072546], PTEX complex [GO:0097619], GO:0097658, plasma membrane protein complex [GO:0098797], outer mitochondrial membrane protein complex [GO:0098799], inner mitochondrial membrane protein complex [GO:0098800], chloroplast thylakoid membrane protein complex [GO:0098807], nuclear membrane protein complex [GO:0106083], COPII vesicles tethering complex [GO:0106103], outer membrane protein complex [GO:0106234], ER-to-endosome phospholipid transfer complex [GO:0140622], PAT complex [GO:0160005], channel complex [GO:0170013], ankyrin-1 complex [GO:0170014], GO:1902495, Bam protein complex [GO:1990063], GO:1990231, Ire1 complex [GO:1990332], GO:1990604, ESCRT IV complex [GO:1990621], GO:1990629, H-gal-GP complex [GO:1990850], GO:1990862 Definition: Any protein complex that is part of a membrane. Relationships: is a type of protein-containing complex [GO:0032991]; is part of membrane [GO:0016020] Sources: GOC:dos